{
  "gene_name": "Formin-2",
  "term_label": "endoplasmic reticulum membrane",
  "gene_symbol": "FMN2",
  "term_id": "GO:0005789",
  "gene": "UniProtKB:Q9NZ56"
}